{
  "term_id": "GO:0035591",
  "gene": "UniProtKB:Q13077",
  "gene_symbol": "TRAF1",
  "term_label": "signaling adaptor activity",
  "gene_name": "TNF receptor-associated factor 1"
}